{
  "gene_symbol": "RPL35",
  "term_label": "maturation of LSU-rRNA from tricistronic rRNA transcript (SSU-rRNA, 5.8S rRNA, LSU-rRNA)",
  "gene_name": "Large ribosomal subunit protein uL29",
  "gene": "UniProtKB:P42766",
  "term_id": "GO:0000463"
}